{
  "term_label": "DNA-binding transcription factor activity, RNA polymerase II-specific",
  "gene_symbol": "NFE2L3",
  "gene": "UniProtKB:Q9Y4A8",
  "gene_name": "Nuclear factor erythroid 2-related factor 3",
  "term_id": "GO:0000981"
}